{
  "gene_symbol": "B4GALNT4",
  "term_label": "Unknown cellular component",
  "gene": "UniProtKB:Q76KP1",
  "term_id": "UNKNOWN:0003",
  "gene_name": "N-acetyl-beta-glucosaminyl-glycoprotein 4-beta-N-acetylgalactosaminyltransferase 1"
}